{
  "gene_name": "Rab GDP dissociation inhibitor beta",
  "term_id": "GO:0016192",
  "gene_symbol": "GDI2",
  "term_label": "vesicle-mediated transport",
  "gene": "UniProtKB:P50395"
}